{
  "gene_symbol": "CDHR3",
  "term_label": "adherens junction",
  "gene": "UniProtKB:Q6ZTQ4",
  "term_id": "GO:0005912",
  "gene_name": "Cadherin-related family member 3"
}